H9 melatonin receptor binding [GO:0031787] (MF) Sources: GOC:mah, GOC:nln Definition: Binding to a H9 melatonin receptor. Relationships: is a type of melatonin receptor binding [GO:0031784] Also known as: H9 melatonin receptor ligand